{
  "gene_symbol": "ATG3",
  "term_label": "glycophagy",
  "term_id": "GO:0061723",
  "gene": "UniProtKB:Q9NT62",
  "gene_name": "Ubiquitin-like-conjugating enzyme ATG3"
}